{
  "gene_symbol": "CDKN2AIP",
  "term_id": "UNKNOWN:0002",
  "gene_name": "CDKN2A-interacting protein",
  "term_label": "Unknown biological process",
  "gene": "UniProtKB:Q9NXV6"
}